glutamyl aminopeptidase activity [GO:0004230] (molecular function) Sources: EC:3.4.11.7 Definition: Catalysis of the release of a N-terminal glutamate (and to a lesser extent aspartate) from a peptide. Relationships: is a type of aminopeptidase activity [GO:0004177] Also known as: Ca2+-activated glutamate aminopeptidase activity, L-aspartate aminopeptidase activity, aminopeptidase A, angiotensinase A, angiotensinase A2, antigen BP-1/6C3 of mouse B lymphocytes, aspartate aminopeptidase activity, glutamyl peptidase activity, membrane aminopeptidase II